{
  "gene_name": "Low-density lipoprotein receptor class A domain-containing protein 4",
  "gene_symbol": "LDLRAD4",
  "term_label": "negative regulation of transforming growth factor beta receptor signaling pathway",
  "term_id": "GO:0030512",
  "gene": "UniProtKB:O15165"
}